{
  "term_id": "GO:0007420",
  "term_label": "brain development",
  "gene_symbol": "AATK",
  "gene": "UniProtKB:Q6ZMQ8",
  "gene_name": "Serine_threonine-protein kinase LMTK1"
}